{
  "gene_symbol": "KBTBD7",
  "term_id": "GO:0005737",
  "gene_name": "Kelch repeat and BTB domain-containing protein 7",
  "term_label": "cytoplasm",
  "gene": "UniProtKB:Q8WVZ9"
}